{
  "gene_symbol": "PRKCB",
  "gene": "UniProtKB:P05771",
  "gene_name": "Protein kinase C beta type",
  "term_label": "Unknown cellular component",
  "term_id": "UNKNOWN:0003"
}